{
  "gene_name": "Protein ecdysoneless homolog",
  "term_id": "UNKNOWN:0002",
  "gene_symbol": "ECD",
  "gene": "UniProtKB:O95905",
  "term_label": "Unknown biological process"
}